determination of left/right symmetry [GO:0007368] (BP) Sources: GOC:dph, GOC:jid Subtypes: GO:0003140, determination of pancreatic left/right asymmetry [GO:0035469], GO:0035545, determination of heart left/right asymmetry [GO:0061371], establishment of left/right asymmetry [GO:0061966], determination of digestive tract left/right asymmetry [GO:0071907], determination of liver left/right asymmetry [GO:0071910], GO:0140969 Definition: The establishment of an organism's body plan or part of an organism with respect to the left and right halves. The pattern can either be symmetric, such that the halves are mirror images, or asymmetric where the pattern deviates from this symmetry. Also known as: determination of left/right asymmetry Relationships: is a type of determination of bilateral symmetry [GO:0009855]; is part of left/right pattern formation [GO:0060972]